rhabdomere membrane biogenesis [GO:0045313] (biological process) Definition: A process that results in the biosynthesis of constituent macromolecules, assembly, and arrangement of constituent parts of a rhabdomere membrane. Sources: GOC:jl Relationships: is a type of membrane biogenesis [GO:0044091]; is part of rhabdomere development [GO:0042052]